negative regulation of positive chemotaxis to cAMP by DIF-1 [GO:0061127] (biological process) Sources: GOC:dph Relationships: is_a regulation of positive chemotaxis to cAMP by DIF-1 [GO:0061120]; is a type of negative regulation of positive chemotaxis to cAMP by chlorinated alkylphenone [GO:0061125] Definition: Any process that decreases the rate, frequency, or extent of directed movement of a motile cell or organism up a concentration gradient of 3',5'-cAMP by the action of DIF-1. DIF-1 is a chlorinated alkylphenone.